{
  "gene": "UniProtKB:Q9UPV9",
  "term_id": "GO:0008333",
  "gene_name": "Trafficking kinesin-binding protein 1",
  "gene_symbol": "TRAK1",
  "term_label": "endosome to lysosome transport"
}